{
  "term_id": "UNKNOWN:0003",
  "gene": "UniProtKB:Q6ZN54",
  "gene_symbol": "DEF8",
  "gene_name": "Differentially expressed in FDCP 8 homolog",
  "term_label": "Unknown cellular component"
}